{
  "term_id": "GO:1990904",
  "gene_name": "Selenocysteine insertion sequence-binding protein 2",
  "gene": "UniProtKB:Q96T21",
  "gene_symbol": "SECISBP2",
  "term_label": "ribonucleoprotein complex"
}